negative regulation of amino acid uptake involved in synaptic transmission [GO:0051942] (biological process) Subtypes: negative regulation of glutamate uptake involved in transmission of nerve impulse [GO:0051948], negative regulation of gamma-aminobutyric acid uptake involved in transmission of nerve impulse [GO:0051949] Also known as: negative regulation of amino acid neurotransmitter reuptake, negative regulation of amino acid neurotransmitter uptake, down regulation of amino acid uptake during transmission of nerve impulse, down-regulation of amino acid uptake during transmission of nerve impulse, downregulation of amino acid uptake during transmission of nerve impulse, inhibition of amino acid uptake during transmission of nerve impulse, negative regulation of amino acid uptake during transmission of nerve impulse Relationships: is a type of GO:0051581; is_a regulation of amino acid uptake involved in synaptic transmission [GO:0051941]; is a type of negative regulation of amino acid transport [GO:0051956]; negatively regulates amino acid neurotransmitter reuptake [GO:0051933] Definition: Any process that stops, prevents, or reduces the frequency, rate or extent of the directed movement of amino acid neurotransmitters into a neuron or glial cell. Sources: GOC:ai